general adaptation syndrome, behavioral process [GO:0051867] (biological process) Sources: GOC:ai Definition: The set of behavioral processes that occur as part of the general adaptation syndrome, the response of the body to a strong, stressful stimulus. Also known as: behavioral process during general adaptation syndrome, behavioral response during general adaptation syndrome, behavioural process during general adaptation syndrome, behavioural response during general adaptation syndrome, general adaptation syndrome, behavioral response, general adaptation syndrome, behavioural process, general adaptation syndrome, behavioural response Relationships: is a type of GO:0007610; is part of general adaptation syndrome [GO:0051866]